{
  "term_label": "nucleus",
  "term_id": "GO:0005634",
  "gene_symbol": "FIGNL2",
  "gene_name": "Fidgetin-like protein 2",
  "gene": "UniProtKB:A6NMB9"
}